imaginal disc eversion [GO:0007561] (biological process) Definition: The eversion (turning inside out) of imaginal discs from their peripodial sacs, resulting in movement of the epithelium to the outside of the larval epidermis. References: PMID:11494317 Relationships: is a type of post-embryonic animal morphogenesis [GO:0009886]; is part of GO:0007560